{
  "gene_symbol": "COA3",
  "term_id": "GO:0033617",
  "term_label": "mitochondrial respiratory chain complex IV assembly",
  "gene": "UniProtKB:Q9Y2R0",
  "gene_name": "Cytochrome c oxidase assembly factor 3 homolog, mitochondrial"
}